inositol hexakisphosphate 4-kinase activity [GO:0000830] (molecular function) Relationships: is a type of inositol hexakisphosphate kinase activity [GO:0000828] Definition: Catalysis of the reaction: ATP + 1D-myo-inositol hexakisphosphate = ADP + 4-diphospho-1D-myo-inositol (1,2,3,5,6)pentakisphosphate. References: PMID:16429326 Sources: GOC:elh